{
  "gene_name": "Major facilitator superfamily domain-containing protein 12",
  "term_id": "GO:0048021",
  "gene": "UniProtKB:Q6NUT3",
  "gene_symbol": "MFSD12",
  "term_label": "regulation of melanin biosynthetic process"
}